{
  "gene": "UniProtKB:Q52LW3",
  "term_id": "GO:0005096",
  "term_label": "GTPase activator activity",
  "gene_symbol": "ARHGAP29",
  "gene_name": "Rho GTPase-activating protein 29"
}